{
  "term_label": "Unknown cellular component",
  "gene_symbol": "ZC2HC1C",
  "gene": "UniProtKB:Q53FD0",
  "gene_name": "Zinc finger C2HC domain-containing protein 1C",
  "term_id": "UNKNOWN:0003"
}